sensory perception of humidity [GO:0098509] (biological process) Also known as: hygrosensory perception Definition: The series of events required for an organism to detect some level of humidity in its environment, convert this detection into a molecular signal, and recognize and characterize the signal. This is a neurological process. Subtypes: sensory perception of high humidity [GO:0098510], sensory perception of low humidity [GO:0098511] Note: Note, this is not classified under 'detection of chemical stimulus' as there are various potential mechanisms of hygroperception including detection of mechanical stimulus. References: PMID:18269908, PMID:8650222 Relationships: is a type of sensory perception [GO:0007600]